{
  "gene": "UniProtKB:A6NDY2",
  "gene_name": "Putative protein FAM90A10",
  "gene_symbol": "FAM90A10",
  "term_id": "UNKNOWN:0003",
  "term_label": "Unknown cellular component"
}